{
  "gene": "UniProtKB:Q8NBF2",
  "term_id": "UNKNOWN:0002",
  "gene_name": "NHL repeat-containing protein 2",
  "term_label": "Unknown biological process",
  "gene_symbol": "NHLRC2"
}